{
  "gene": "UniProtKB:Q96T17",
  "gene_name": "MAP7 domain-containing protein 2",
  "term_label": "microtubule cytoskeleton",
  "term_id": "GO:0015630",
  "gene_symbol": "MAP7D2"
}